{
  "gene_name": "Large ribosomal subunit protein uL14m",
  "gene": "UniProtKB:Q6P1L8",
  "term_label": "mitochondrion",
  "term_id": "GO:0005739",
  "gene_symbol": "MRPL14"
}